{
  "gene_symbol": "THAP12",
  "term_label": "Unknown cellular component",
  "gene": "UniProtKB:O43422",
  "gene_name": "52 kDa repressor of the inhibitor of the protein kinase",
  "term_id": "UNKNOWN:0003"
}